{
  "gene": "UniProtKB:Q8HWS3",
  "gene_name": "DNA-binding protein RFX6",
  "term_label": "endocrine pancreas development",
  "term_id": "GO:0031018",
  "gene_symbol": "RFX6"
}